germacrene C synthase activity [GO:0102904] (molecular function) Sources: EC:4.2.3.60, GOC:pz Relationships: is a type of carbon-oxygen lyase activity, acting on phosphates [GO:0016838] Definition: Catalysis of the reaction: 2-trans,6-trans-farnesyl diphosphate = germacrene C + diphosphoric acid.